regulation of filamentous growth of a population of unicellular organisms in response to biotic stimulus [GO:1900443] (biological process) Definition: Any process that modulates the frequency, rate or extent of filamentous growth of a population of unicellular organisms in response to biotic stimulus. Sources: GOC:TermGenie, GOC:di Subtypes: negative regulation of filamentous growth of a population of unicellular organisms in response to biotic stimulus [GO:1900444], positive regulation of filamentous growth of a population of unicellular organisms in response to biotic stimulus [GO:1900445] Relationships: is a type of regulation of response to biotic stimulus [GO:0002831]; is a type of regulation of filamentous growth of a population of unicellular organisms [GO:1900428]; regulates filamentous growth of a population of unicellular organisms in response to biotic stimulus [GO:0036180]